{
  "gene_symbol": "DCDC1",
  "gene_name": "Doublecortin domain-containing protein 1",
  "gene": "UniProtKB:M0R2J8",
  "term_id": "GO:0008017",
  "term_label": "microtubule binding"
}